{
  "gene_name": "Thioredoxin domain-containing protein 12",
  "term_id": "UNKNOWN:0002",
  "gene_symbol": "TXNDC12",
  "gene": "UniProtKB:O95881",
  "term_label": "Unknown biological process"
}